nucleoside bisphosphate catabolic process [GO:0033869] (biological process) Sources: GOC:mah, GOC:pde Also known as: nucleoside bisphosphate breakdown, nucleoside bisphosphate catabolism, nucleoside bisphosphate degradation Definition: The chemical reactions and pathways resulting in the breakdown of a nucleoside bisphosphate, a compound consisting of a nucleobase linked to a deoxyribose or ribose sugar esterified with one phosphate group attached to each of two different hydroxyl groups on the sugar. Relationships: is a type of nucleoside bisphosphate metabolic process [GO:0033865]; is a type of nucleoside phosphate catabolic process [GO:1901292] Subtypes: ribonucleoside bisphosphate catabolic process [GO:0034031], purine nucleoside bisphosphate catabolic process [GO:0034034]